{
  "gene": "UniProtKB:Q6ZW05",
  "term_id": "UNKNOWN:0002",
  "gene_name": "Patched domain-containing protein 4",
  "gene_symbol": "PTCHD4",
  "term_label": "Unknown biological process"
}